{
  "term_label": "nucleolus",
  "gene": "UniProtKB:Q9NXV6",
  "term_id": "GO:0005730",
  "gene_symbol": "CDKN2AIP",
  "gene_name": "CDKN2A-interacting protein"
}